{
  "term_id": "GO:0000978",
  "gene_symbol": "NHLH2",
  "term_label": "RNA polymerase II cis-regulatory region sequence-specific DNA binding",
  "gene": "UniProtKB:Q02577",
  "gene_name": "Helix-loop-helix protein 2"
}